{
  "gene": "UniProtKB:Q86XE3",
  "term_id": "GO:0005509",
  "gene_symbol": "MICU3",
  "gene_name": "Calcium uptake protein 3, mitochondrial",
  "term_label": "calcium ion binding"
}